{
  "gene_name": "Putative C-type lectin domain family 20 member A",
  "term_id": "UNKNOWN:0003",
  "gene_symbol": "CLEC20A",
  "gene": "UniProtKB:Q6ZU45",
  "term_label": "Unknown cellular component"
}